{
  "gene_symbol": "RSPO3",
  "term_id": "GO:0005615",
  "term_label": "extracellular space",
  "gene": "UniProtKB:Q9BXY4",
  "gene_name": "R-spondin-3"
}